radial spoke base 1 [GO:0120340] (cellular component) References: PMID:22754630, PMID:25694453 Sources: GOC:krc Relationships: is a type of radial spoke base [GO:0120339]; BFO_0000050 radial spoke 1 [GO:0120333] Definition: The short portion of the radial spoke 1 (RS1) that is directly anchored to the A microtubule of an axonemal microtubule doublet.